exocrine pancreas development [GO:0031017] (biological process) Sources: GOC:cvs Relationships: is a type of GO:0048732; is part of pancreas development [GO:0031016]; is part of exocrine system development [GO:0035272]; is part of digestive system development [GO:0055123] Definition: The process whose specific outcome is the progression of the exocrine pancreas over time, from its formation to the mature structure. The exocrine pancreas produces and store zymogens of digestive enzymes, such as chymotrypsinogen and trypsinogen in the acinar cells.